{
  "term_label": "metalloendopeptidase activity",
  "gene_name": "A disintegrin and metalloproteinase with thrombospondin motifs 13",
  "gene_symbol": "ADAMTS13",
  "gene": "UniProtKB:Q76LX8",
  "term_id": "GO:0004222"
}